{
  "term_label": "cytoplasm",
  "gene_name": "Cysteine protease ATG4A",
  "gene_symbol": "ATG4A",
  "term_id": "GO:0005737",
  "gene": "UniProtKB:Q8WYN0"
}